{
  "gene_name": "Paired-like homeodomain transcription factor LEUTX",
  "gene_symbol": "LEUTX",
  "gene": "UniProtKB:A8MZ59",
  "term_label": "DNA-binding transcription factor activity, RNA polymerase II-specific",
  "term_id": "GO:0000981"
}